{
  "gene_name": "Pro-FMRFamide-related neuropeptide VF",
  "gene_symbol": "NPVF",
  "gene": "UniProtKB:Q9HCQ7",
  "term_label": "Unknown cellular component",
  "term_id": "UNKNOWN:0003"
}